gamma-guanidinobutyraldehyde dehydrogenase (NAD+) activity [GO:0047107] (MF) Relationships: is a type of aldehyde dehydrogenase (NAD+) activity [GO:0004029] Also known as: 4-guanidinobutanal:NAD+ 1-oxidoreductase activity, 4-guanidinobutyraldehyde dehydrogenase activity, GBAL dehydrogenase activity, alpha-guanidinobutyraldehyde dehydrogenase activity Definition: Catalysis of the reaction: 4-guanidinobutanal + H2O + NAD+ = 4-guanidinobutanoate + 2 H+ + NADH. Sources: RHEA:14381